{
  "gene_name": "UL16-binding protein 1",
  "gene": "UniProtKB:Q9BZM6",
  "term_label": "antigen processing and presentation of endogenous peptide antigen via MHC class I via ER pathway, TAP-independent",
  "term_id": "GO:0002486",
  "gene_symbol": "ULBP1"
}